{
  "gene": "UniProtKB:Q6PIZ9",
  "gene_symbol": "TRAT1",
  "gene_name": "T-cell receptor-associated transmembrane adapter 1",
  "term_label": "negative regulation of receptor recycling",
  "term_id": "GO:0001920"
}